{
  "gene": "UniProtKB:Q96N68",
  "gene_name": "Putative uncharacterized protein C18orf15",
  "term_label": "Unknown cellular component",
  "term_id": "UNKNOWN:0003",
  "gene_symbol": "C18orf15"
}